{
  "gene_name": "Chromaffin granule amine transporter",
  "gene_symbol": "SLC18A1",
  "term_id": "GO:0030672",
  "term_label": "synaptic vesicle membrane",
  "gene": "UniProtKB:P54219"
}